protein localization to nuclear body [GO:1903405] (biological process) Definition: A process in which a protein is transported to, or maintained in, a location within a nuclear body. References: PMID:24713849 Sources: GOC:TermGenie, GO_REF:0000087 Also known as: protein localisation in nuclear body, protein localisation to nuclear body, protein localization in nuclear body Relationships: is a type of GO:1990173 Subtypes: GO:1904867